{
  "gene": "UniProtKB:Q9UGM1",
  "term_label": "regulation of membrane potential",
  "gene_name": "Neuronal acetylcholine receptor subunit alpha-9",
  "gene_symbol": "CHRNA9",
  "term_id": "GO:0042391"
}